{
  "gene": "UniProtKB:Q9BS86",
  "term_label": "Unknown molecular function",
  "term_id": "UNKNOWN:0001",
  "gene_symbol": "ZPBP",
  "gene_name": "Zona pellucida-binding protein 1"
}